regulation of proteolysis associated with antigen processing and presentation [GO:0002628] (BP) Subtypes: negative regulation of proteolysis associated with antigen processing and presentation [GO:0002629], positive regulation of proteolysis associated with antigen processing and presentation [GO:0002630] Relationships: is a type of regulation of proteolysis involved in protein catabolic process [GO:1903050]; RO_0002211 proteolysis associated with antigen processing and presentation [GO:0002496] Sources: GOC:add Definition: Any process that modulates the frequency, rate, or extent of proteolysis associated with antigen processing and presentation.